{
  "term_id": "GO:0005634",
  "gene_name": "RNA-binding motif, single-stranded-interacting protein 1",
  "gene_symbol": "RBMS1",
  "term_label": "nucleus",
  "gene": "UniProtKB:P29558"
}